{
  "gene": "UniProtKB:Q9H7P6",
  "term_label": "regulation of epidermal growth factor receptor signaling pathway",
  "gene_name": "Multivesicular body subunit 12B",
  "term_id": "GO:0042058",
  "gene_symbol": "MVB12B"
}